maintenance of bipolar cell polarity regulating cell shape [GO:0061305] (BP) Sources: GOC:dph, GOC:vw Relationships: is a type of establishment or maintenance of bipolar cell polarity regulating cell shape [GO:0061246] Definition: The maintenance of established bipolar anisotropic intracellular organization or cell growth patterns that results in the shaping of a cell. Regulation: positively regulated by positive regulation of maintenance of bipolar cell polarity regulating cell shape [GO:0061361]; negatively regulated by GO:0061362; regulated by GO:2000115